{
  "term_id": "UNKNOWN:0001",
  "term_label": "Unknown molecular function",
  "gene_name": "T cell receptor beta variable 29-1",
  "gene_symbol": "TRBV29-1",
  "gene": "UniProtKB:A0A5B7"
}